microtubule bundle [GO:0097427] (cellular component) Sources: NIF_Subcellular:sao1872343973 Relationships: is a type of cellular anatomical structure [GO:0110165]; is part of cytoskeleton [GO:0005856]; has part GO:0005874 Subtypes: static microtubule bundle [GO:0099070], dynamic microtubule bundle [GO:0099071], axon microtubule bundle [GO:1901589], GO:1905720 Definition: An arrangement of closely apposed microtubules running parallel to each other. Also known as: microtubule fascicle